{
  "gene_symbol": "COL1A2",
  "term_id": "GO:0031012",
  "gene_name": "Collagen alpha-2(I) chain",
  "gene": "UniProtKB:P08123",
  "term_label": "extracellular matrix"
}